lipid import into cell [GO:0140354] (biological process) Also known as: lipid uptake Relationships: is a type of lipid transport [GO:0006869] Subtypes: long-chain fatty acid import into cell [GO:0044539], vitamin A import into cell [GO:0071939] Sources: GOC:pg Definition: The directed movement of a lipid from outside of a cell into a cell. This may occur via transport across the plasma membrane or via endocytosis.